positive regulation of heat generation [GO:0031652] (biological process) Subtypes: positive regulation of fever generation [GO:0031622] Sources: GOC:dph, GOC:mah, GOC:tb Definition: Any process that activates or increases the rate or extent of heat generation. Also known as: up regulation of heat generation, up-regulation of heat generation, upregulation of heat generation, activation of heat generation, stimulation of heat generation Relationships: is a type of regulation of heat generation [GO:0031650]; is a type of positive regulation of multicellular organismal process [GO:0051240]; positively regulates heat generation [GO:0031649]